aorta morphogenesis [GO:0035909] (BP) Definition: The process in which the anatomical structures of an aorta are generated and organized. An aorta is an artery that carries blood from the heart to other parts of the body. Sources: GOC:bf, GOC:dgh, MA:0000062, UBERON:0000947, Wikipedia:Aorta Subtypes: dorsal aorta morphogenesis [GO:0035912], ventral aorta morphogenesis [GO:0035913] Regulation: regulated by regulation of aorta morphogenesis [GO:1903847]; negatively regulated by negative regulation of aorta morphogenesis [GO:1903848]; positively regulated by positive regulation of aorta morphogenesis [GO:1903849] Relationships: is a type of artery morphogenesis [GO:0048844]; is part of aorta development [GO:0035904]